{
  "term_label": "protein-containing complex",
  "gene_name": "Lymphocyte antigen 6 complex locus protein G6c",
  "gene_symbol": "LY6G6C",
  "gene": "UniProtKB:O95867",
  "term_id": "GO:0032991"
}